{
  "gene": "UniProtKB:Q9H410",
  "term_id": "GO:0000444",
  "term_label": "MIS12/MIND type complex",
  "gene_symbol": "DSN1",
  "gene_name": "Kinetochore-associated protein DSN1 homolog"
}